{
  "gene": "UniProtKB:Q969E8",
  "gene_symbol": "TSR2",
  "gene_name": "Pre-rRNA-processing protein TSR2 homolog",
  "term_label": "nucleus",
  "term_id": "GO:0005634"
}